positive regulation of protein targeting to membrane [GO:0090314] (biological process) Relationships: is a type of positive regulation of cellular process [GO:0048522]; is a type of GO:0090313; is a type of positive regulation of establishment of protein localization [GO:1904951]; positively regulates protein targeting to membrane [GO:0006612] Subtypes: GO:1900485 Sources: GOC:tb Definition: Any process that increases the frequency, rate or extent of the process of directing proteins towards a membrane, usually using signals contained within the protein.